lncRNA transcription [GO:0140742] (biological process) Definition: The transcription of lncRNAs, non-coding RNAs over 200 nucleotides in length, from a DNA template. References: PMID:33767452, PMID:33913806 Relationships: is a type of DNA-templated transcription [GO:0006351] Regulation: regulated by GO:0140743; negatively regulated by negative regulation of lncRNA transcription [GO:0140744]